{
  "term_label": "DNA-binding transcription factor activity, RNA polymerase II-specific",
  "term_id": "GO:0000981",
  "gene_symbol": "NEUROD1",
  "gene": "UniProtKB:Q13562",
  "gene_name": "Neurogenic differentiation factor 1"
}